{
  "gene_name": "D-amino-acid oxidase",
  "gene_symbol": "DAO",
  "gene": "UniProtKB:P14920",
  "term_id": "GO:0055130",
  "term_label": "D-alanine catabolic process"
}